hydroxyacid-oxoacid transhydrogenase activity [GO:0047988] (molecular function) Also known as: (S)-3-hydroxybutanoate:2-oxoglutarate oxidoreductase activity, transhydrogenase, hydroxy acid-oxo acid Relationships: is a type of oxidoreductase activity, acting on CH-OH group of donors [GO:0016614] Sources: EC:1.1.99.24, MetaCyc:HYDROXYACID-OXOACID-TRANSHYDROGENASE-RXN Definition: Catalysis of the reaction: (S)-3-hydroxybutanoate + 2-oxoglutarate = acetoacetate + (R)-2-hydroxyglutarate.